{
  "term_id": "GO:0016779",
  "gene_symbol": "YRDC",
  "term_label": "nucleotidyltransferase activity",
  "gene_name": "Threonylcarbamoyl-AMP synthase",
  "gene": "UniProtKB:Q86U90"
}